{
  "gene_name": "Forkhead box protein S1",
  "term_id": "GO:0006357",
  "gene": "UniProtKB:O43638",
  "gene_symbol": "FOXS1",
  "term_label": "regulation of transcription by RNA polymerase II"
}